neural nucleus development [GO:0048857] (BP) Subtypes: locus ceruleus development [GO:0021703], inferior olivary nucleus development [GO:0021713], superior olivary nucleus development [GO:0021718], GO:0021724, superior raphe nucleus development [GO:0021725], lateral reticular nucleus development [GO:0021726], GO:0021728, trigeminal sensory nucleus development [GO:0021730], trigeminal motor nucleus development [GO:0021731], GO:0021735, globose nucleus development [GO:0021736], emboliform nucleus development [GO:0021737], fastigial nucleus development [GO:0021738], abducens nucleus development [GO:0021742], hypoglossal nucleus development [GO:0021743], GO:0021744, nucleus ambiguus development [GO:0021745], GO:0021746, cochlear nucleus development [GO:0021747], vestibular nucleus development [GO:0021750], salivary nucleus development [GO:0021751], GO:0021754, caudate nucleus development [GO:0021757], GO:0021758, globus pallidus development [GO:0021759], substantia nigra development [GO:0021762], subthalamic nucleus development [GO:0021763], GO:0021768, lateral geniculate nucleus development [GO:0021771], GO:0061451 Relationships: is a type of anatomical structure development [GO:0048856] Sources: GO_REF:0000021 Definition: The biological process whose specific outcome is the progression of a neural nucleus from its initial condition to its mature state. A neural nucleus is an anatomical structure consisting of a discrete aggregate of neuronal soma.